{
  "gene": "UniProtKB:P17600",
  "gene_name": "Synapsin-1",
  "term_id": "GO:0097091",
  "gene_symbol": "SYN1",
  "term_label": "synaptic vesicle clustering"
}